{
  "gene_name": "Cyclin-dependent kinases regulatory subunit 2",
  "gene_symbol": "CKS2",
  "term_label": "cyclin-dependent protein serine/threonine kinase activator activity",
  "term_id": "GO:0061575",
  "gene": "UniProtKB:P33552"
}